interleukin-5 receptor activity [GO:0004914] (molecular function) Also known as: IL-5 receptor activity, IL-5R Relationships: is_a cytokine receptor activity [GO:0004896]; is part of interleukin-5-mediated signaling pathway [GO:0038043]; has part interleukin-5 binding [GO:0019980] Definition: Combining with interleukin-5 and transmitting the signal from one side of the membrane to the other to initiate a change in cell activity. Sources: GOC:jl, GOC:signaling